centriole-centriole cohesion [GO:0010457] (biological process) Definition: The cell cycle process in which the two centrioles within a centrosome remain tightly paired. Relationships: is a type of cell cycle process [GO:0022402]; is part of centrosome cycle [GO:0007098] Regulation: regulated by regulation of centriole-centriole cohesion [GO:0030997]; negatively regulated by GO:1903126; positively regulated by positive regulation of centriole-centriole cohesion [GO:1903127] Sources: GOC:dph, GOC:tb